autophagosome membrane [GO:0000421] (cellular component) Definition: The lipid bilayer surrounding an autophagosome, a double-membrane-bounded vesicle in which endogenous cellular material is sequestered. Sources: GOC:autophagy, GOC:isa_complete Subtypes: GO:1904930 Also known as: autophagic vacuole membrane Relationships: is a type of GO:0005774; is part of autophagosome [GO:0005776]